{
  "term_id": "GO:0019369",
  "gene_symbol": "CYP4F2",
  "term_label": "arachidonate metabolic process",
  "gene_name": "Cytochrome P450 4F2",
  "gene": "UniProtKB:P78329"
}